{
  "term_label": "positive regulation of cell migration",
  "term_id": "GO:0030335",
  "gene_name": "Eotaxin",
  "gene": "UniProtKB:P51671",
  "gene_symbol": "CCL11"
}